antibacterial peptide biosynthetic process [GO:0002780] (biological process) References: PMID:11807545, PMID:15638771 Sources: GOC:add, ISBN:0781735149 Definition: The chemical reactions and pathways resulting in the formation of an antibacterial peptide. Relationships: is a type of antimicrobial peptide biosynthetic process [GO:0002777]; is part of antibacterial peptide production [GO:0002778] Regulation: regulated by regulation of antibacterial peptide biosynthetic process [GO:0002808]; negatively regulated by GO:0002809; positively regulated by GO:0006963 Subtypes: biosynthetic process of antibacterial peptides active against Gram-negative bacteria [GO:0002812], biosynthetic process of antibacterial peptides active against Gram-positive bacteria [GO:0002815]